negative regulation of toll-like receptor 10 signaling pathway [GO:0034168] (biological process) Also known as: negative regulation of TLR10 signaling pathway, negative regulation of toll-like receptor 10 signalling pathway Definition: Any process that stops, prevents, or reduces the frequency, rate, or extent of toll-like receptor 10 signaling pathway. Relationships: is a type of negative regulation of immune system process [GO:0002683]; is a type of negative regulation of signal transduction [GO:0009968]; is a type of GO:0034167; negatively regulates toll-like receptor 10 signaling pathway [GO:0034166] References: PMID:16551253, PMID:17328678 Sources: GOC:add